{
  "term_id": "UNKNOWN:0003",
  "gene_name": "Olfactory receptor 5H8",
  "gene_symbol": "OR5H8",
  "term_label": "Unknown cellular component",
  "gene": "UniProtKB:P0DN80"
}